NADPH dehydrogenase (quinone) activity [GO:0008753] (molecular function) Sources: RHEA:46164 Definition: Catalysis of the reaction: NADPH + H+ + a quinone = NADP+ + a quinol. Also known as: NADPH oxidase, NADPH:(quinone-acceptor) oxidoreductase, reduced nicotinamide adenine dinucleotide phosphate (quinone) dehydrogenase Relationships: is_a GO:0003955; is a type of NADPH dehydrogenase activity [GO:0003959]